regulation of gluconeogenesis [GO:0006111] (biological process) Also known as: regulation of glucose biosynthesis, regulation of glucose biosynthetic process, regulation of gluconeogenesis involved in cellular glucose homeostasis Sources: GOC:go_curators Subtypes: negative regulation of gluconeogenesis [GO:0045721], positive regulation of gluconeogenesis [GO:0045722] Definition: Any process that modulates the frequency, rate or extent of gluconeogenesis, the formation of glucose from noncarbohydrate precursors, such as pyruvate, amino acids and glycerol. Relationships: is a type of regulation of glucose metabolic process [GO:0010906]; is a type of regulation of carbohydrate biosynthetic process [GO:0043255]; RO_0002211 gluconeogenesis [GO:0006094]